4-hydroxy-3-methylbut-2-en-1-yl diphosphate synthase activity (ferredoxin) [GO:0046429] (molecular function) Definition: Catalysis of the reaction: (E)-4-hydroxy-3-methylbut-2-en-1-yl diphosphate + H2O + 2 oxidized ferredoxin = 2-C-methyl-D-erythritol 2,4-cyclodiphosphate + 2 reduced ferredoxin. Relationships: is a type of GO:0052592 Also known as: (E)-4-hydroxy-3-methylbut-2-enyl diphosphate synthase activity, 1-hydroxy-2-methyl-2-(E)-butenyl 4-diphosphate synthase activity, 1-hydroxy-2-methyl-2-butenyl 4-diphosphate synthase activity, (E)-4-hydroxy-3-methylbut-2-en-1-yl-diphosphate:oxidized ferredoxin oxidoreductase activity References: PMID:11752431 Sources: EC:1.17.7.1